precatalytic spliceosome [GO:0071011] (cellular component) Definition: A spliceosomal complex that is formed by the recruitment of a preassembled U5-containing tri-snRNP to the prespliceosome. Although all 5 snRNPs are present, the precatalytic spliceosome is catalytically inactive. The precatalytic spliceosome includes many proteins in addition to those found in the associated snRNPs. Relationships: is a type of GO:0005681 Subtypes: U2-type precatalytic spliceosome [GO:0071005], GO:0071016 References: PMID:18322460, PMID:19239890 Sources: GOC:ab, GOC:krc, GOC:mah Also known as: mammalian spliceosomal complex B, mammalian spliceosomal complex B1, yeast spliceosomal complex A2-1